interleukin-6-mediated signaling pathway [GO:0070102] (BP) Sources: GOC:BHF, GOC:add, GOC:mah, GOC:signaling Relationships: is a type of GO:0019221; is part of cellular response to interleukin-6 [GO:0071354] Regulation: regulated by regulation of interleukin-6-mediated signaling pathway [GO:0070103]; negatively regulated by negative regulation of interleukin-6-mediated signaling pathway [GO:0070104]; positively regulated by positive regulation of interleukin-6-mediated signaling pathway [GO:0070105] Also known as: interleukin-6-mediated signalling pathway, IL-6-mediated signaling pathway Definition: The series of molecular signals initiated by interleukin-6 binding to a receptor on the surface of a target cell, and ending with the regulation of a downstream cellular process, e.g. transcription.